{
  "gene": "UniProtKB:Q13015",
  "term_id": "GO:0005829",
  "term_label": "cytosol",
  "gene_name": "Protein AF1q",
  "gene_symbol": "MLLT11"
}